{
  "gene_symbol": "CLDN18",
  "term_id": "UNKNOWN:0001",
  "term_label": "Unknown molecular function",
  "gene": "UniProtKB:P56856",
  "gene_name": "Claudin-18"
}